memory T cell activation [GO:0035709] (biological process) Sources: CL:0000813, GOC:BHF Definition: The change in morphology and behavior of a memory T cell resulting from exposure to a mitogen, cytokine, chemokine, cellular ligand, or an antigen for which it is specific. Relationships: is a type of T cell activation [GO:0042110] Regulation: regulated by regulation of memory T cell activation [GO:2000567]; positively regulated by positive regulation of memory T cell activation [GO:2000568]